cyanosome [GO:0043701] (cellular component) Definition: A tissue-specific, membrane-bounded cytoplasmic organelle within which an unknown blue pigment is localized. Cyanosomes are synthesized in cyanophores and are blue in appearance. Relationships: is a type of GO:0048770 Sources: GOC:mh